acetyl-CoA biosynthetic process from ethanol [GO:0019431] (BP) Definition: The chemical reactions and pathways resulting in the formation of acetyl-CoA from ethanol via acetaldehyde. Sources: GOC:go_curators Also known as: acetyl-CoA anabolism from ethanol, acetyl-CoA formation from ethanol, acetyl-CoA synthesis from ethanol Relationships: is a type of GO:0006067; is_a acetyl-CoA biosynthetic process [GO:0006085]; is a type of generation of precursor metabolites and energy [GO:0006091]